{
  "term_id": "GO:0005634",
  "gene": "UniProtKB:Q9BQF6",
  "gene_symbol": "SENP7",
  "gene_name": "Sentrin-specific protease 7",
  "term_label": "nucleus"
}